positive regulation of amphiregulin production [GO:0140732] (biological process) Relationships: is a type of GO:0001819; is a type of regulation of amphiregulin production [GO:0140731]; positively regulates amphiregulin production [GO:0140730] Also known as: positive regulation of AREG production References: PMID:24463227 Definition: Any process that activates or increases the frequency, rate or extent of production of amphiregulin.